{
  "term_id": "GO:0019158",
  "gene_symbol": "HK3",
  "gene_name": "Hexokinase-3",
  "gene": "UniProtKB:P52790",
  "term_label": "mannokinase activity"
}